{
  "gene_name": "Protein lifeguard 3",
  "term_id": "GO:0005783",
  "gene_symbol": "TMBIM1",
  "term_label": "endoplasmic reticulum",
  "gene": "UniProtKB:Q969X1"
}